{
  "gene_name": "TBC1 domain family member 3I",
  "gene": "UniProtKB:A0A087WXS9",
  "gene_symbol": "TBC1D3I",
  "term_label": "Unknown biological process",
  "term_id": "UNKNOWN:0002"
}